{
  "gene": "UniProtKB:O94986",
  "gene_name": "Centrosomal protein of 152 kDa",
  "gene_symbol": "CEP152",
  "term_label": "centriole replication",
  "term_id": "GO:0007099"
}